{
  "gene_symbol": "TAAR2",
  "gene_name": "Trace amine-associated receptor 2",
  "term_label": "trace-amine receptor activity",
  "gene": "UniProtKB:Q9P1P5",
  "term_id": "GO:0001594"
}